{
  "gene": "UniProtKB:Q8N4X5",
  "gene_symbol": "AFAP1L2",
  "gene_name": "Actin filament-associated protein 1-like 2",
  "term_id": "GO:0007346",
  "term_label": "regulation of mitotic cell cycle"
}